{
  "term_label": "anatomical structure morphogenesis",
  "term_id": "GO:0009653",
  "gene_symbol": "PITX1",
  "gene_name": "Pituitary homeobox 1",
  "gene": "UniProtKB:P78337"
}